{
  "gene": "UniProtKB:Q9NPQ8",
  "term_label": "cytoplasm",
  "gene_symbol": "RIC8A",
  "gene_name": "Synembryn-A",
  "term_id": "GO:0005737"
}